{
  "gene_name": "Nuclear receptor subfamily 0 group B member 1",
  "gene_symbol": "NR0B1",
  "term_id": "GO:0000122",
  "term_label": "negative regulation of transcription by RNA polymerase II",
  "gene": "UniProtKB:P51843"
}